ciliary pro-basal body [GO:0120280] (cellular component) Definition: The cilary pro-basal body is an immature, partially assembled form of a ciliary basal body found next to the basal body of a cilium. Pro-basal bodies are not capable of nucleating a cilium. As the cell progresses through the cell cycle, continuing assembly will convert the pro-basal body into a mature basal body that is capable of nucleating a cilium. Note: Pro-basal bodies are distinct from basal bodies as they are not at the base of a cilium and are not capable of nucleating a cilium. While immature, they contain some structures in common with the mature basal body and also may contain proteins unique to the immature state. Note that cilia and eukaryotic flagella are deemed to be equivalent. In many eukaryotic cells, 'ciliary basal body' (GO:0036064) and 'centriole' (GO:0005814) represent a common entity that cycles through its function in cell division, then ciliogenesis, then cell division again. However, these structures are modified extensively as they transition into each other, and may contain different proteins, specific to each component. In other eukaryotic cells, centrioles are not involved in cell division but only in cilium assembly, which is thought to be the ancestral role of the centriole/basal body. Sources: ISBN:0198547684 Also known as: pro-basal body, pro-centriole, probasal body, flagellar pro-basal body, flagellar probasal body Relationships: is a type of cellular anatomical structure [GO:0110165]